{
  "gene_name": "Signal transducing adapter molecule 2",
  "term_id": "GO:0007165",
  "gene_symbol": "STAM2",
  "term_label": "signal transduction",
  "gene": "UniProtKB:O75886"
}